{
  "gene_symbol": "ZSCAN30",
  "term_label": "Unknown cellular component",
  "gene": "UniProtKB:Q86W11",
  "gene_name": "Zinc finger and SCAN domain-containing protein 30",
  "term_id": "UNKNOWN:0003"
}